{
  "gene_symbol": "ERBB4",
  "gene_name": "Receptor tyrosine-protein kinase erbB-4",
  "term_label": "negative regulation of apoptotic process",
  "gene": "UniProtKB:Q15303",
  "term_id": "GO:0043066"
}